{
  "gene_symbol": "FYN",
  "term_id": "GO:0005886",
  "gene": "UniProtKB:P06241",
  "term_label": "plasma membrane",
  "gene_name": "Tyrosine-protein kinase Fyn"
}